{
  "gene_name": "Enoyl-CoA hydratase, mitochondrial",
  "gene": "UniProtKB:P30084",
  "term_id": "GO:0006635",
  "term_label": "fatty acid beta-oxidation",
  "gene_symbol": "ECHS1"
}